{
  "gene": "UniProtKB:P48742",
  "gene_symbol": "LHX1",
  "term_label": "RNA polymerase II transcription regulatory region sequence-specific DNA binding",
  "gene_name": "LIM_homeobox protein Lhx1",
  "term_id": "GO:0000977"
}